{
  "term_id": "GO:0005737",
  "gene_name": "Mitogen-activated protein kinase kinase kinase 9",
  "gene_symbol": "MAP3K9",
  "gene": "UniProtKB:P80192",
  "term_label": "cytoplasm"
}